{
  "gene_symbol": "ZDHHC15",
  "gene_name": "Palmitoyltransferase ZDHHC15",
  "gene": "UniProtKB:Q96MV8",
  "term_label": "protein targeting to membrane",
  "term_id": "GO:0006612"
}